{
  "term_label": "membrane",
  "gene": "UniProtKB:P0C7Q6",
  "gene_name": "Solute carrier family 35 member G6",
  "term_id": "GO:0016020",
  "gene_symbol": "SLC35G6"
}